{
  "term_id": "UNKNOWN:0001",
  "gene_name": "DNA repair protein XRCC4",
  "gene_symbol": "XRCC4",
  "term_label": "Unknown molecular function",
  "gene": "UniProtKB:Q13426"
}